{
  "gene_symbol": "KLK4",
  "gene_name": "Kallikrein-4",
  "term_id": "GO:0004252",
  "term_label": "serine-type endopeptidase activity",
  "gene": "UniProtKB:Q9Y5K2"
}